{
  "gene_symbol": "HSPA14",
  "term_label": "ribosome",
  "gene": "UniProtKB:Q0VDF9",
  "term_id": "GO:0005840",
  "gene_name": "Heat shock 70 kDa protein 14"
}